{
  "gene": "UniProtKB:O95235",
  "term_id": "GO:0016887",
  "term_label": "ATP hydrolysis activity",
  "gene_name": "Kinesin-like protein KIF20A",
  "gene_symbol": "KIF20A"
}